positive regulation of compound eye retinal cell programmed cell death [GO:0046672] (biological process) Relationships: is a type of GO:0046669; is a type of positive regulation of retinal cell programmed cell death [GO:0046670]; positively regulates compound eye retinal cell programmed cell death [GO:0046667] Sources: GOC:ai Also known as: activation of retinal cell programmed cell death, positive regulation of retinal cell programmed cell death, stimulation of retinal cell programmed cell death, up regulation of retinal cell programmed cell death, up-regulation of retinal cell programmed cell death, upregulation of retinal cell programmed cell death Subtypes: GO:1901694 Definition: Any process that activates or increases the frequency, rate or extent of programmed cell death that occurs in the compound eye retina.